methylthiol:coenzyme M methyltransferase activity [GO:0044683] (molecular function) Note: This reaction is achieved by the catalysis of two successive steps carried out by the same enzyme - the transfer of a methyl group from the substrate to the cobalt cofactor of a methylated-thiol-specific corrinoid protein (MtsB), and the subsequent transfer of the methyl group from the corrinoid protein to coenzyme M. With most other methanogenesis substrates this process is carried out by two different enzymes (for example, EC:2.1.1.90, methanol-corrinoid protein Co-methyltransferase, and EC:2.1.1.246, methylated methanol-specific corrinoid protein:coenzyme M methyltransferase). The cobalt is oxidized during methylation from the Co(I) state to the Co(III) state, and is reduced back to the Co(I) form during demethylation. Relationships: is_a methyltransferase activity [GO:0008168] References: PMID:9371433 Sources: MetaCyc:RXN-8125 Definition: Catalysis of the overall reaction: methyl-Co(III) methylated-thiol-specific corrinoid protein + coenzyme M = Co(I) methylated--thiol-specific corrinoid protein + methyl-CoM. Also known as: methylthiol:coenzyme M methyl transferase activity